{
  "gene_name": "Vesicular integral-membrane protein VIP36",
  "term_label": "COPII-coated ER to Golgi transport vesicle",
  "gene_symbol": "LMAN2",
  "term_id": "GO:0030134",
  "gene": "UniProtKB:Q12907"
}